{
  "gene_name": "Dipeptidase 3",
  "gene_symbol": "DPEP3",
  "gene": "UniProtKB:Q9H4B8",
  "term_id": "UNKNOWN:0002",
  "term_label": "Unknown biological process"
}